aspartate transmembrane import into vacuole [GO:0090453] (biological process) Sources: GOC:tb Definition: The directed movement of aspartate into the vacuole across the vacuolar membrane. Also known as: vacuolar aspartate import Relationships: is a type of aspartate transmembrane transport [GO:0015810]; is a type of vacuolar transmembrane transport [GO:0034486]; is_a vacuolar amino acid transmembrane transport [GO:0034487]